transcription initiation at mitochondrial promoter [GO:0006391] (biological process) Relationships: is a type of mitochondrial RNA metabolic process [GO:0000959]; is a type of GO:0006352; BFO_0000050 mitochondrial transcription [GO:0006390] References: PMID:33127643 Also known as: transcription initiation from mitochondrial promoter Definition: A transcription initiation process that takes place at a promoter on the mitochondrial chromosome.